{
  "term_id": "GO:0000307",
  "gene_symbol": "CDK6",
  "gene": "UniProtKB:Q00534",
  "term_label": "cyclin-dependent protein kinase holoenzyme complex",
  "gene_name": "Cyclin-dependent kinase 6"
}